UDP-N,N'-diacetylbacillosamine 2-epimerase activity [GO:0102388] (molecular function) Sources: EC:3.2.1.184, GOC:pz Definition: Catalysis of the reaction: UDP-N,N'-diacetylbacillosamine + H2O = 2,4-diacetamido-2,4,6-trideoxy-alpha-D-mannopyranose + UDP + H+. Relationships: is a type of hydrolase activity, hydrolyzing O-glycosyl compounds [GO:0004553]